{
  "gene_symbol": "TRAV39",
  "gene_name": "T cell receptor alpha variable 39",
  "gene": "UniProtKB:A0A0B4J263",
  "term_id": "UNKNOWN:0003",
  "term_label": "Unknown cellular component"
}